regulation of Golgi vesicle fusion to target membrane [GO:0048214] (biological process) Definition: Any process that modulates the frequency, rate or extent of Golgi vesicle fusion to target membrane. References: PMID:10219233 Sources: GOC:jid, ISBN:0716731363 Note: Note that GTP-binding Rab proteins serve as regulators of vesicle targeting and fusion. Relationships: is a type of regulation of vesicle fusion [GO:0031338]; regulates Golgi vesicle fusion to target membrane [GO:0048210] Subtypes: positive regulation of Golgi vesicle fusion to target membrane [GO:0048215], GO:0048216